{
  "term_label": "oligosaccharide metabolic process",
  "term_id": "GO:0009311",
  "gene_name": "Sia-alpha-2,3-Gal-beta-1,4-GlcNAc-R:alpha 2,8-sialyltransferase",
  "gene": "UniProtKB:O43173",
  "gene_symbol": "ST8SIA3"
}